{
  "gene": "UniProtKB:O75154",
  "term_id": "GO:0030139",
  "term_label": "endocytic vesicle",
  "gene_name": "Rab11 family-interacting protein 3",
  "gene_symbol": "RAB11FIP3"
}